{
  "gene_name": "Toll-like receptor 9",
  "term_label": "defense response to virus",
  "term_id": "GO:0051607",
  "gene_symbol": "TLR9",
  "gene": "UniProtKB:Q9NR96"
}